{
  "term_label": "low-density lipoprotein particle binding",
  "term_id": "GO:0030169",
  "gene_name": "Collectin-12",
  "gene": "UniProtKB:Q5KU26",
  "gene_symbol": "COLEC12"
}